phthalate 4,5-dioxygenase activity [GO:0018620] (molecular function) Relationships: is a type of GO:0016708 Sources: EC:1.14.12.7, RHEA:17489 Also known as: phthalate dioxygenase activity, PDO activity, phthalate,NADH:oxygen oxidoreductase (4,5-hydroxylating) Definition: Catalysis of the reaction: H+ + NADH + O2 + phthalate = cis-4,5-dihydroxycyclohexa-2,6-diene-1,2-dicarboxylate + NAD+.